{
  "term_label": "intracellular signal transduction",
  "gene_name": "Serine_threonine-protein kinase N1",
  "term_id": "GO:0035556",
  "gene_symbol": "PKN1",
  "gene": "UniProtKB:Q16512"
}